{
  "term_label": "innate immune response in mucosa",
  "gene_name": "Histone H2B type 1-C_E_F_G_I",
  "term_id": "GO:0002227",
  "gene_symbol": "H2BC10",
  "gene": "UniProtKB:P62807"
}